tRNA threonylcarbamoyladenosine dehydratase [GO:0061503] (molecular function) Relationships: is a type of hydro-lyase activity [GO:0016836]; is a type of GO:0140101 Definition: Catalysis of the ATP-dependent dehydration of t6A to form cyclic t6A. References: PMID:23242255 Sources: GOC:dph